{
  "gene": "UniProtKB:P13611",
  "term_id": "UNKNOWN:0001",
  "gene_name": "Versican core protein",
  "term_label": "Unknown molecular function",
  "gene_symbol": "VCAN"
}